regulation of vascular permeability [GO:0043114] (biological process) Sources: GOC:jl Definition: Any process that modulates the extent to which blood vessels can be pervaded by fluid. Subtypes: GO:0002528, negative regulation of vascular permeability [GO:0043116], positive regulation of vascular permeability [GO:0043117], regulation of blood-brain barrier permeability [GO:1905603], regulation of lymphatic vascular permeability [GO:1990185] Relationships: is a type of vascular process in circulatory system [GO:0003018]; is a type of regulation of biological quality [GO:0065008]; is part of blood circulation [GO:0008015]